{
  "term_label": "molybdopterin cofactor metabolic process",
  "gene_symbol": "MOCOS",
  "term_id": "GO:0043545",
  "gene": "UniProtKB:Q96EN8",
  "gene_name": "Molybdenum cofactor sulfurase"
}